{
  "gene": "UniProtKB:P62380",
  "term_label": "Unknown cellular component",
  "term_id": "UNKNOWN:0003",
  "gene_symbol": "TBPL1",
  "gene_name": "TATA box-binding protein-like 1"
}